{
  "term_label": "synaptic vesicle docking",
  "term_id": "GO:0016081",
  "gene_symbol": "RIMS1",
  "gene": "UniProtKB:Q86UR5",
  "gene_name": "Regulating synaptic membrane exocytosis protein 1"
}